{
  "gene_symbol": "TOPBP1",
  "gene": "UniProtKB:Q92547",
  "term_id": "GO:0006270",
  "gene_name": "DNA topoisomerase 2-binding protein 1",
  "term_label": "DNA replication initiation"
}